{
  "gene_symbol": "CDH9",
  "gene_name": "Cadherin-9",
  "term_id": "GO:0044331",
  "gene": "UniProtKB:Q9ULB4",
  "term_label": "cell-cell adhesion mediated by cadherin"
}